{
  "term_label": "Unknown biological process",
  "gene_name": "NADH dehydrogenase [ubiquinone] 1 beta subcomplex subunit 3",
  "gene_symbol": "NDUFB3",
  "term_id": "UNKNOWN:0002",
  "gene": "UniProtKB:O43676"
}